{
  "term_id": "UNKNOWN:0003",
  "gene_symbol": "GOLGA6L22",
  "gene_name": "Golgin subfamily A member 6-like protein 22",
  "term_label": "Unknown cellular component",
  "gene": "UniProtKB:H0YM25"
}